{
  "gene_symbol": "ZKSCAN8P1",
  "term_id": "UNKNOWN:0001",
  "term_label": "Unknown molecular function",
  "gene": "UniProtKB:A0A8I5KTY6",
  "gene_name": "HCG1646484"
}